{
  "gene": "UniProtKB:Q15172",
  "term_label": "protein phosphatase type 2A complex",
  "gene_name": "Serine_threonine-protein phosphatase 2A 56 kDa regulatory subunit alpha isoform",
  "term_id": "GO:0000159",
  "gene_symbol": "PPP2R5A"
}